{
  "term_label": "RNA 7-methylguanosine cap binding",
  "gene_name": "Eukaryotic translation initiation factor 4E",
  "gene": "UniProtKB:P06730",
  "term_id": "GO:0000340",
  "gene_symbol": "EIF4E"
}